epithelial cell migration involved in proximal tubule morphogenesis [GO:0072159] (biological process) Definition: The orderly movement of epithelial cells within a renal tubule that contributes to proximal tubule morphogenesis. Relationships: is a type of GO:0072155; is part of proximal tubule morphogenesis [GO:0072158] Subtypes: epithelial cell migration involved in mesonephric proximal tubule morphogenesis [GO:0061280], epithelial cell migration involved in metanephric proximal tubule morphogenesis [GO:0072292] Sources: GOC:mtg_kidney_jan10